{
  "gene": "UniProtKB:Q8TE49",
  "term_id": "GO:0005737",
  "gene_name": "OTU domain-containing protein 7A",
  "gene_symbol": "OTUD7A",
  "term_label": "cytoplasm"
}